{
  "gene_symbol": "RPL27",
  "term_id": "GO:0022625",
  "gene_name": "Large ribosomal subunit protein eL27",
  "term_label": "cytosolic large ribosomal subunit",
  "gene": "UniProtKB:P61353"
}